{
  "gene": "UniProtKB:Q8WVV5",
  "gene_name": "Butyrophilin subfamily 2 member A2",
  "gene_symbol": "BTN2A2",
  "term_label": "regulation of cytokine production",
  "term_id": "GO:0001817"
}